{
  "term_id": "UNKNOWN:0001",
  "term_label": "Unknown molecular function",
  "gene_symbol": "C19orf73",
  "gene": "UniProtKB:Q9NVV2",
  "gene_name": "Putative uncharacterized protein C19orf73"
}